{
  "gene": "UniProtKB:P33527",
  "gene_symbol": "ABCC1",
  "term_label": "carboxylic acid transmembrane transporter activity",
  "gene_name": "Multidrug resistance-associated protein 1",
  "term_id": "GO:0046943"
}